{
  "term_label": "immunoglobulin mediated immune response",
  "term_id": "GO:0016064",
  "gene_symbol": "IGHV4-4",
  "gene": "UniProtKB:A0A075B6R2",
  "gene_name": "Immunoglobulin heavy variable 4-4"
}